{
  "gene_name": "Phosphatidylinositol 4,5-bisphosphate 3-kinase catalytic subunit alpha isoform",
  "term_id": "GO:0016477",
  "gene": "UniProtKB:P42336",
  "term_label": "cell migration",
  "gene_symbol": "PIK3CA"
}